{
  "gene_name": "Myeloid leukemia factor 2",
  "gene_symbol": "MLF2",
  "gene": "UniProtKB:Q15773",
  "term_id": "GO:0006355",
  "term_label": "regulation of DNA-templated transcription"
}